{
  "term_id": "GO:0061630",
  "gene_symbol": "RNF43",
  "gene": "UniProtKB:Q68DV7",
  "gene_name": "E3 ubiquitin-protein ligase RNF43",
  "term_label": "ubiquitin protein ligase activity"
}